{
  "gene_name": "Protein BTG3",
  "gene": "UniProtKB:Q14201",
  "term_id": "UNKNOWN:0001",
  "term_label": "Unknown molecular function",
  "gene_symbol": "BTG3"
}